regulation of gastric emptying [GO:0120060] (biological process) Relationships: is a type of GO:1905333; regulates GO:0035483 Also known as: regulation of small bowel emptying, regulation of small intestine emptying References: PMID:15890336 Sources: GOC:sl Subtypes: negative regulation of gastric emptying [GO:0120061], positive regulation of gastric emptying [GO:0120062] Definition: Any process that modulates the frequency, rate or extent of any gastric emptying process, the process in which the liquid and liquid-suspended solid contents of the stomach exit through the pylorus into the duodenum.